autophagosome-membrane adaptor activity [GO:0160183] (molecular function) Definition: The binding activity of a molecule that brings together a target membrane and an autophagosome during autophagy. References: PMID:30544615, PMID:36635405 Relationships: is a type of protein-membrane adaptor activity [GO:0043495]; is a type of GO:0160247 Subtypes: GO:0140506, mitochondrion autophagosome adaptor activity [GO:0140580]